formaldehyde dehydrogenase (NAD+) activity [GO:0018467] (molecular function) Sources: RHEA:16425 Relationships: is a type of aldehyde dehydrogenase (NAD+) activity [GO:0004029] Definition: Catalysis of the reaction: formaldehyde + H2O + NAD+ = formate + 2 H+ + NADH. Also known as: glutathione-independent formaldehyde dehydrogenase activity, formaldehyde:NAD+ oxidoreductase activity